histone H4K12 methyltransferase activity [GO:0140984] (molecular function) Definition: Catalysis of the reaction: S-adenosyl-L-methionine + histone H4 L-lysine (position 12) = S-adenosyl-L-homocysteine + histone H4 N6-methyl-L-lysine (position 12). This reaction is the addition of a methyl group to the lysine residue at position 12 of the histone H4 protein. References: PMID:12086618 Relationships: is a type of protein-lysine N-methyltransferase activity [GO:0016279]; is a type of histone H4 methyltransferase activity [GO:0140939] Also known as: histone H4K12 methylase activity, histone H4 lysine 12-specific methyltransferase activity, histone H4K12 methylation, histone lysine N-methyltransferase activity (H4-K12 specific), histone methylase activity (H4-K12 specific), histone methyltransferase activity (H4-K12 specific), histone-H4K12 methyltransferase activity Note: Note that the residue position corresponds to the canonical human H4 histone (UniProtKB:P02309); this residue is conserved across all eukaryotes. Note that the initiation methionine is cleaved, so the first residue is S1.